{
  "term_label": "nicotinic acid receptor activity",
  "gene_symbol": "HCAR2",
  "term_id": "GO:0070553",
  "gene": "UniProtKB:Q8TDS4",
  "gene_name": "Hydroxycarboxylic acid receptor 2"
}